negative regulation of DNA strand resection involved in replication fork processing [GO:0110027] (BP) References: PMID:28475874 Sources: GOC:mah Definition: Any process that stops, prevents, or reduces the frequency, rate or extent of DNA strand resection involved in replication fork processing. Relationships: is_a regulation of DNA strand resection involved in replication fork processing [GO:0110026]; is a type of negative regulation of DNA-templated DNA replication [GO:2000104]; negatively regulates DNA strand resection involved in replication fork processing [GO:0110025]